{
  "gene_name": "DNA-binding protein inhibitor ID-1",
  "gene_symbol": "ID1",
  "term_id": "GO:0030182",
  "gene": "UniProtKB:P41134",
  "term_label": "neuron differentiation"
}